{
  "gene_name": "Rho-related BTB domain-containing protein 1",
  "term_id": "GO:0003924",
  "term_label": "GTPase activity",
  "gene_symbol": "RHOBTB1",
  "gene": "UniProtKB:O94844"
}